{
  "gene_symbol": "TAF12",
  "gene_name": "Transcription initiation factor TFIID subunit 12",
  "gene": "UniProtKB:Q16514",
  "term_id": "GO:0005669",
  "term_label": "transcription factor TFIID complex"
}